fatty acid synthase complex [GO:0005835] (cellular component) Definition: A multienzyme complex that catalyses the synthesis of fatty acids from acetyl CoA. Relationships: is a type of intracellular protein-containing complex [GO:0140535]; is_a catalytic complex [GO:1902494] Also known as: FAS complex, cytosolic FAS complex, cytosolic fatty acid synthase complex, cytosolic type I FAS complex, cytosolic type I fatty acid synthase complex, fatty acid synthetase complex, holo-[acyl-carrier-protein] synthase complex Sources: GOC:pde, GOC:sgd_curators, ISBN:0716746840